{
  "term_id": "UNKNOWN:0002",
  "gene_symbol": "TMEM35B",
  "term_label": "Unknown biological process",
  "gene": "UniProtKB:Q8NCS4",
  "gene_name": "Transmembrane protein 35B"
}